{
  "term_label": "single-stranded DNA binding",
  "gene_symbol": "MCM2",
  "term_id": "GO:0003697",
  "gene_name": "DNA replication licensing factor MCM2",
  "gene": "UniProtKB:P49736"
}